11alpha-30-dihydroxy beta-amyrin dehydrogenase activity [GO:0102369] (molecular function) Relationships: is a type of oxidoreductase activity, acting on paired donors, with incorporation or reduction of molecular oxygen [GO:0016705] Sources: GOC:pz Definition: Catalysis of the reaction: 11alpha,30-dihydroxy-beta-amyrin + NADPH + O2 + H+ = 30-hydroxy-11-oxo-beta-amyrin + NADP + 2 H2O.